gamma-aminobutyric acid:sodium:chloride symporter activity [GO:0005332] (MF) Definition: Enables the transfer of a solute or solutes from one side of a membrane to the other according to the reaction: gamma-aminobutyric acid(out) + Na+(out) + Cl-(out) = gamma-aminobutyric acid(in) + Na+(in) + Cl(in). References: PMID:7589472, PMID:7861179 Also known as: sodium/chloride-dependent GABA transporter activity, 4-aminobutanoate:sodium symporter activity, 4-aminobutyrate:sodium symporter activity, GABA:sodium symporter activity, betaine/GABA:sodium symporter activity, gamma-aminobutyric acid:sodium symporter activity Note: See also the molecular function term 'neurotransmitter:sodium symporter activity ; GO:0005328'. Relationships: is a type of amino acid:sodium symporter activity [GO:0005283]; is a type of gamma-aminobutyric acid transmembrane transporter activity [GO:0015185]; is a type of GO:0015378; is a type of monocarboxylate:sodium symporter activity [GO:0140161]